{
  "term_id": "UNKNOWN:0002",
  "gene_symbol": "ZMAT1",
  "gene_name": "Zinc finger matrin-type protein 1",
  "gene": "UniProtKB:Q5H9K5",
  "term_label": "Unknown biological process"
}